{
  "gene": "UniProtKB:P51956",
  "term_label": "Unknown biological process",
  "gene_symbol": "NEK3",
  "term_id": "UNKNOWN:0002",
  "gene_name": "Serine_threonine-protein kinase Nek3"
}